{
  "gene": "UniProtKB:P23229",
  "gene_symbol": "ITGA6",
  "term_id": "GO:0034676",
  "gene_name": "Integrin alpha-6",
  "term_label": "integrin alpha6-beta4 complex"
}